{
  "term_label": "tRNA binding",
  "gene": "UniProtKB:Q9BY44",
  "gene_symbol": "EIF2A",
  "gene_name": "Eukaryotic translation initiation factor 2A",
  "term_id": "GO:0000049"
}